{
  "term_id": "GO:0050852",
  "gene": "UniProtKB:P78410",
  "gene_name": "Butyrophilin subfamily 3 member A2",
  "gene_symbol": "BTN3A2",
  "term_label": "T cell receptor signaling pathway"
}